{
  "term_id": "GO:0000981",
  "term_label": "DNA-binding transcription factor activity, RNA polymerase II-specific",
  "gene_name": "Zinc finger protein 142",
  "gene_symbol": "ZNF142",
  "gene": "UniProtKB:P52746"
}